{
  "gene_symbol": "CDCA8",
  "term_id": "GO:0000070",
  "gene": "UniProtKB:Q53HL2",
  "gene_name": "Borealin",
  "term_label": "mitotic sister chromatid segregation"
}